{
  "gene_name": "Probable non-functional immunoglobulin heavy variable 8-51-1",
  "gene": "UniProtKB:P0DTE2",
  "gene_symbol": "IGHV8-51-1",
  "term_id": "GO:0016064",
  "term_label": "immunoglobulin mediated immune response"
}